{
  "gene_symbol": "DUSP9",
  "gene_name": "Dual specificity protein phosphatase 9",
  "term_id": "GO:0005737",
  "term_label": "cytoplasm",
  "gene": "UniProtKB:Q99956"
}